{
  "gene_symbol": "MESP2",
  "gene_name": "Mesoderm posterior protein 2",
  "gene": "UniProtKB:Q0VG99",
  "term_id": "GO:0006357",
  "term_label": "regulation of transcription by RNA polymerase II"
}